{
  "gene_symbol": "SGPL1",
  "term_id": "GO:0005783",
  "term_label": "endoplasmic reticulum",
  "gene_name": "Sphingosine-1-phosphate lyase 1",
  "gene": "UniProtKB:O95470"
}